lipid metabolic process [GO:0006629] (biological process) Also known as: lipid metabolism Relationships: is a type of GO:0044238 Regulation: RO_0002211 by regulation of lipid metabolic process [GO:0019216]; negatively regulated by negative regulation of lipid metabolic process [GO:0045833]; positively regulated by GO:0045834 Definition: The chemical reactions and pathways involving lipids, compounds soluble in an organic solvent but not, or sparingly, in an aqueous solvent. Includes fatty acids; neutral fats, other fatty-acid esters, and soaps; long-chain (fatty) alcohols and waxes; sphingoids and other long-chain bases; glycolipids, phospholipids and sphingolipids; and carotenes, polyprenols, sterols, terpenes and other isoprenoids. Sources: GOC:ma Subtypes: fatty acid metabolic process [GO:0006631], neutral lipid metabolic process [GO:0006638], GO:0006643, GO:0006644, isoprenoid metabolic process [GO:0006720], steroid metabolic process [GO:0008202], lipid biosynthetic process [GO:0008610], lipid catabolic process [GO:0016042], lipid modification [GO:0030258], ether lipid metabolic process [GO:0046485], glycerolipid metabolic process [GO:0046486], GO:0046505, fatty acid derivative metabolic process [GO:1901568], liposaccharide metabolic process [GO:1903509]